{
  "term_label": "Unknown biological process",
  "gene_symbol": "NPIPB6",
  "term_id": "UNKNOWN:0002",
  "gene_name": "Nuclear pore complex-interacting protein family member B6",
  "gene": "UniProtKB:E9PJ23"
}